R8 cell-mediated photoreceptor organization [GO:0045470] (biological process) References: PMID:11880339 Relationships: is a type of regionalization [GO:0003002]; is part of compound eye photoreceptor development [GO:0042051] Definition: The regionalization process that coordinates the recruitment and organization of other non-R8 photoreceptors by the R8 photoreceptor. Also known as: R8-mediated photoreceptor organisation